{
  "term_label": "olfactory receptor activity",
  "gene_symbol": "OR13D1",
  "term_id": "GO:0004984",
  "gene_name": "Olfactory receptor 13D1",
  "gene": "UniProtKB:Q8NGV5"
}